{
  "term_label": "receptor antagonist activity",
  "gene_name": "Dickkopf-related protein 4",
  "gene": "UniProtKB:Q9UBT3",
  "term_id": "GO:0048019",
  "gene_symbol": "DKK4"
}